astral microtubule nucleation [GO:0030954] (biological process) Definition: The 'de novo' formation of an astral microtubule, in which tubulin heterodimers form metastable oligomeric aggregates, some of which go on to support formation of a complete microtubule. Sources: GOC:mah Relationships: is a type of astral microtubule organization [GO:0030953]; is a type of microtubule nucleation by microtubule organizing center [GO:0051418]